{
  "gene_symbol": "GZMA",
  "term_id": "GO:0004252",
  "gene": "UniProtKB:P12544",
  "term_label": "serine-type endopeptidase activity",
  "gene_name": "Granzyme A"
}